methanophenazine biosynthetic process [GO:1900630] (biological process) Also known as: methanophenazine anabolism, methanophenazine biosynthesis, methanophenazine formation, methanophenazine synthesis Regulation: regulated by GO:1900962; negatively regulated by negative regulation of methanophenazine biosynthetic process [GO:1900963]; positively regulated by positive regulation of methanophenazine biosynthetic process [GO:1900964] Sources: GOC:TermGenie, GOC:mengo_curators Relationships: is a type of biosynthetic process [GO:0009058]; is a type of methanophenazine metabolic process [GO:1900629] Definition: The chemical reactions and pathways resulting in the formation of methanophenazine.